{
  "gene_name": "C-C motif chemokine 20",
  "gene": "UniProtKB:P78556",
  "term_label": "Unknown biological process",
  "term_id": "UNKNOWN:0002",
  "gene_symbol": "CCL20"
}